{
  "gene_symbol": "PRR30",
  "gene": "UniProtKB:Q53SZ7",
  "term_id": "UNKNOWN:0001",
  "gene_name": "Proline-rich protein 30",
  "term_label": "Unknown molecular function"
}